oxalate decarboxylase activity [GO:0046564] (molecular function) Definition: Catalysis of the reaction: H+ + oxalate = CO2 + formate. Sources: EC:4.1.1.2, RHEA:16509 Relationships: is a type of GO:0016831 Also known as: oxalate carboxy-lyase (formate-forming), oxalate carboxy-lyase activity